chemokine (C-C motif) ligand 2 signaling pathway [GO:0038148] (biological process) Subtypes: CCL2-activated CCR2 signaling pathway [GO:0038151], CCL2-activated CCR4 signaling pathway [GO:0038153] Sources: GOC:nhn, GOC:signaling, Wikipedia:CCL2 Also known as: CCL2 signaling pathway Definition: The series of molecular signals initiated by the binding of the C-C chemokine CCL2 to its receptor on the surface of a target cell, and ending with the regulation of a downstream cellular process, e.g. transcription. Relationships: is a type of GO:0070098